interleukin-7 receptor complex [GO:1905540] (cellular component) References: PMID:19141282 Sources: GOC:TermGenie, GOC:bhm, GO_REF:0000088 Also known as: IL-7 receptor complex, IL-7-receptor complex, IL7 receptor complex, IL7-receptor complex Definition: A protein complex that binds interleukin-7 (IL-7) and that consists of, at a minimum, an interleukin, an alpha and a gamma chain as well as optional additional kinase subunits. The alpha chain binds IL-7 with high affinity and subsequently binds the cytokine receptor common gamma chain that forms part of multiple interleukin receptors. Note: An example of this is IL7R in human (P16871) in PMID:19141282 (inferred from direct assay). Relationships: is a type of GO:0043235